sporangium development [GO:0043582] (biological process) Definition: The process whose specific outcome is the progression of the sporangium over time, from its formation to the mature structure. A sporangium is a structure producing and containing spores. Regulation: regulated by GO:0075310; positively regulated by positive regulation of sporangium development [GO:0075311]; negatively regulated by GO:0075312 Also known as: sporangia development Relationships: is a type of spore-bearing structure development [GO:0075259] Sources: GOC:jl, Wikipedia:Sporagium Subtypes: GO:0075222, oomycete sporangium development [GO:0075321]